{
  "term_label": "aminoacyl-tRNA synthetase multienzyme complex",
  "gene_name": "Lysine--tRNA ligase",
  "gene_symbol": "KARS1",
  "term_id": "GO:0017101",
  "gene": "UniProtKB:Q15046"
}